phagosome-lysosome docking [GO:0090384] (biological process) Sources: GOC:kmv, GOC:tb Definition: The initial attachment of a phagosome membrane to a lysosome membrane. Docking requires only that the proteins come close enough to interact and adhere. Subtypes: phagosome-lysosome docking involved in apoptotic cell clearance [GO:0090388] Also known as: lysosome recruitment to phagosome Relationships: is a type of GO:0048278; is part of GO:0001845